{
  "term_id": "GO:0070888",
  "gene_symbol": "OLIG1",
  "term_label": "E-box binding",
  "gene_name": "Oligodendrocyte transcription factor 1",
  "gene": "UniProtKB:Q8TAK6"
}